pronephric glomerulus morphogenesis [GO:0035775] (biological process) Definition: The process in which the anatomical structures of the pronephric glomerulus are generated and organized. The pronephric glomerulus is part of the pronephric nephron and is restricted to one body segment. References: PMID:18787069 Sources: GOC:mtg_kidney_jan10, GOC:yaf Note: This term is intended for annotation of fish and other organisms which contain a glomerulus as part of the pronephric nephron. It should not be used for annotation of Xenopus, which contains a pronephric glomus rather than a glomerulus. Relationships: is a type of GO:0072102; is part of pronephric glomerulus development [GO:0039021]